{
  "gene_symbol": "LRIG1",
  "term_label": "sensory perception of sound",
  "gene_name": "Leucine-rich repeats and immunoglobulin-like domains protein 1",
  "gene": "UniProtKB:Q96JA1",
  "term_id": "GO:0007605"
}